{
  "gene_symbol": "AKNA",
  "gene_name": "Microtubule organization protein AKNA",
  "term_id": "GO:0060234",
  "gene": "UniProtKB:Q7Z591",
  "term_label": "neuroblast delamination"
}